{
  "term_label": "Unknown molecular function",
  "term_id": "UNKNOWN:0001",
  "gene_name": "Membrane frizzled-related protein",
  "gene": "UniProtKB:Q9BY79",
  "gene_symbol": "MFRP"
}